{
  "gene_name": "Histone-lysine N-methyltransferase SETMAR",
  "gene_symbol": "SETMAR",
  "gene": "UniProtKB:Q53H47",
  "term_id": "GO:0042800",
  "term_label": "histone H3K4 methyltransferase activity"
}